cellobiose catabolic process [GO:2000892] (biological process) Regulation: regulated by regulation of cellobiose catabolic process [GO:1900282]; negatively regulated by negative regulation of cellobiose catabolic process [GO:1900283]; positively regulated by positive regulation of cellobiose catabolic process [GO:1900284] Sources: GOC:mengo_curators Definition: The chemical reactions and pathways resulting in the breakdown of a cellobiose. Relationships: is_a disaccharide catabolic process [GO:0046352]; is a type of cellobiose metabolic process [GO:2000891] Also known as: cellobiose catabolism